dolichylphosphate-glucose phosphodiesterase activity [GO:0047397] (molecular function) Relationships: is a type of phosphoric diester hydrolase activity [GO:0008081] Sources: EC:3.1.4.48, MetaCyc:3.1.4.48-RXN Also known as: dolichyl-phosphate-glucose phosphodiesterase activity, Dol-P-Glc phosphodiesterase activity, dolichol phosphoglucose phosphodiesterase activity, dolichyl-beta-D-glucosyl-phosphate dolichylphosphohydrolase activity Definition: Catalysis of the reaction: dolichyl beta-D-glucosyl phosphate + H2O = dolichol-phosphate + beta-D-glucose.